establishment of cell polarity regulating cell shape [GO:0071964] (biological process) Regulation: regulated by regulation of establishment of cell polarity regulating cell shape [GO:2000782]; negatively regulated by negative regulation of establishment of cell polarity regulating cell shape [GO:2000783]; positively regulated by positive regulation of establishment of cell polarity regulating cell shape [GO:2000784] Sources: GOC:mah Definition: Any cellular process that results in the specification or formation of a polarized intracellular organization or cell growth pattern that regulates the shape of a cell. Relationships: is a type of establishment of cell polarity [GO:0030010]; is a type of establishment or maintenance of cell polarity regulating cell shape [GO:0071963]